{
  "gene_name": "Electrogenic sodium bicarbonate cotransporter 4",
  "term_id": "GO:0008510",
  "gene": "UniProtKB:Q9BY07",
  "gene_symbol": "SLC4A5",
  "term_label": "sodium:bicarbonate symporter activity"
}